{
  "gene_name": "Synaptotagmin-5",
  "term_id": "GO:0070382",
  "term_label": "exocytic vesicle",
  "gene_symbol": "SYT5",
  "gene": "UniProtKB:O00445"
}